dendritic cell homeostasis [GO:0036145] (biological process) Also known as: DC homeostasis Relationships: is a type of leukocyte homeostasis [GO:0001776] Definition: The process of regulating the proliferation and elimination of dendritic cells such that the total number of dendritic cells within a whole or part of an organism is stable over time in the absence of an outside stimulus. References: PMID:12570827, PMID:19176316 Sources: CL:0000451, GOC:uh